maltose-6'-phosphate glucosidase activity [GO:0050081] (MF) Relationships: is a type of GO:0015926 Also known as: maltose-6'-phosphate 6-phosphoglucohydrolase activity, phospho-alpha-glucosidase activity Definition: Catalysis of the reaction: H2O + maltose 6'-phosphate = D-glucose + D-glucose 6-phosphate. Sources: EC:3.2.1.122, MetaCyc:MALTOSE-6-PHOSPHATE-GLUCOSIDASE-RXN